{
  "gene_symbol": "CD27",
  "term_label": "Unknown molecular function",
  "gene": "UniProtKB:P26842",
  "term_id": "UNKNOWN:0001",
  "gene_name": "CD27 antigen"
}